carbohydrate derivative transport [GO:1901264] (biological process) Relationships: is a type of transport [GO:0006810] Subtypes: hexose phosphate transport [GO:0015712], triose phosphate transport [GO:0015717], N-acetylgalactosamine transport [GO:0015763], N-acetylglucosamine transport [GO:0015764], GO:0015777, GO:0015780, GO:0015794, peptidoglycan transport [GO:0015835], GO:0015858, purine ribonucleotide transport [GO:0015868], nicotinamide mononucleotide transport [GO:0015890], lipopolysaccharide transport [GO:0015920], deoxynucleotide transport [GO:0030302], glycoprotein transport [GO:0034436], glycolipid transport [GO:0046836], GO:0051977, glycerol-2-phosphate transmembrane transport [GO:0070811], glucosinolate transport [GO:1901349], GO:1901656, N,N'-diacetylchitobiose import [GO:1902815], 5-amino-1-ribofuranosylimidazole-4-carboxamide transmembrane transport [GO:1903088] Definition: The directed movement of a carbohydrate derivative into, out of or within a cell, or between cells, by means of some agent such as a transporter or pore. Sources: GOC:TermGenie, GOC:bf, GOC:jl